{
  "gene_name": "Transcriptional repressor protein YY1",
  "term_id": "GO:0000785",
  "term_label": "chromatin",
  "gene": "UniProtKB:P25490",
  "gene_symbol": "YY1"
}